{
  "gene_symbol": "ABCA7",
  "gene_name": "Phospholipid-transporting ATPase ABCA7",
  "term_label": "phosphatidylcholine floppase activity",
  "gene": "UniProtKB:Q8IZY2",
  "term_id": "GO:0090554"
}